{
  "gene_name": "Putative ankyrin repeat domain-containing protein 20A4",
  "term_label": "Unknown molecular function",
  "term_id": "UNKNOWN:0001",
  "gene": "UniProtKB:Q4UJ75",
  "gene_symbol": "ANKRD20A4P"
}